{
  "gene_name": "Protein LTO1 homolog",
  "term_label": "Unknown cellular component",
  "term_id": "UNKNOWN:0003",
  "gene": "UniProtKB:Q8WV07",
  "gene_symbol": "LTO1"
}